pterinosome [GO:0043700] (cellular component) Relationships: is a type of GO:0048770 Definition: A tissue-specific, membrane-bounded cytoplasmic organelle within which pteridine pigments are synthesized and stored. Pterinosomes are synthesized in xanthophores and erythrophore cells and are yellow, orange or red in appearance. Sources: GOC:mh